tracheary element differentiation [GO:1905177] (biological process) Definition: The process in which a relatively unspecialized cell acquires the specialized features of a tracheary element. References: PMID:20659276 Sources: GOC:TermGenie, GO_REF:0000086 Relationships: is a type of cell differentiation [GO:0030154] Subtypes: xylem vessel member cell differentiation [GO:0048759]